{
  "gene_name": "Stabilizer of axonemal microtubules 2",
  "gene": "UniProtKB:Q658L1",
  "term_id": "UNKNOWN:0002",
  "gene_symbol": "SAXO2",
  "term_label": "Unknown biological process"
}